negative regulation of antimicrobial humoral response [GO:0008348] (biological process) Definition: Any process that stops, prevents, or reduces the frequency, rate, or extent of an antimicrobial humoral response. Sources: GOC:go_curators Subtypes: negative regulation of antimicrobial peptide production [GO:0002785] Relationships: is a type of regulation of antimicrobial humoral response [GO:0002759]; is a type of negative regulation of response to biotic stimulus [GO:0002832]; is a type of negative regulation of humoral immune response [GO:0002921]; is a type of GO:0031348; is a type of negative regulation of response to external stimulus [GO:0032102]; negatively regulates antimicrobial humoral response [GO:0019730] Also known as: attenuation of antimicrobial humoral response, down regulation of antimicrobial humoral response, down-regulation of antimicrobial humoral response, downregulation of antimicrobial humoral response, inhibition of antimicrobial humoral response